{
  "term_label": "cytoplasm",
  "term_id": "GO:0005737",
  "gene_symbol": "TDP2",
  "gene_name": "Tyrosyl-DNA phosphodiesterase 2",
  "gene": "UniProtKB:O95551"
}